CMP biosynthetic process [GO:0009224] (biological process) Sources: ISBN:0198506732 Definition: The chemical reactions and pathways resulting in the formation of CMP, cytidine monophosphate. Relationships: is a type of pyrimidine ribonucleoside monophosphate biosynthetic process [GO:0009174]; is a type of pyrimidine ribonucleotide biosynthetic process [GO:0009220]; is a type of GO:0046035 Also known as: CMP anabolism, CMP biosynthesis, CMP formation, CMP synthesis Subtypes: CMP salvage [GO:0006238]